{
  "term_id": "GO:0042554",
  "gene_symbol": "NCF1B",
  "gene_name": "Putative neutrophil cytosol factor 1B",
  "term_label": "superoxide anion generation",
  "gene": "UniProtKB:A6NI72"
}